modulation of penetration peg formation [GO:0075054] (biological process) Subtypes: GO:0075055 Relationships: is a type of regulation of developmental process [GO:0050793]; is_a modulation by symbiont of entry into host [GO:0052372]; regulates penetration peg formation [GO:0075053] Sources: GOC:pamgo_curators Note: Note that this term should not be used to annotate gene products of the host. It should only be used to annotate those gene products from the symbiont involved in this process. Also known as: modulation of symbiont penetration peg formation for entry into host, modulation of symbiont penetration peg initiation Definition: Any process that modulates the frequency, rate or extent of symbiont penetration peg formation for entry into host. The host is defined as the larger of the organisms involved in a symbiotic interaction.